U6atac snRNP [GO:0005691] (cellular component) Relationships: is a type of spliceosomal snRNP complex [GO:0097525] Also known as: snRNP U6atac Sources: GOC:krc, GOC:mah, ISBN:0879695897 Definition: A ribonucleoprotein complex that contains small nuclear RNA U6atac, the Lsm2-8 heptameric ring complex, as well as several proteins that are unique to the U6atac snRNP, most of which remain associated with the U6atac snRNA both while the U6atac snRNP is free or assembled into the U4atac/U6atac snRNP or into a series of spliceosomal complexes.